{
  "gene": "UniProtKB:Q5T280",
  "term_label": "kinetochore",
  "gene_name": "Putative methyltransferase C9orf114",
  "term_id": "GO:0000776",
  "gene_symbol": "SPOUT1"
}